negative regulation of galactomannan catabolic process [GO:2000992] (biological process) Relationships: is a type of negative regulation of catabolic process [GO:0009895]; is a type of GO:0010605; is a type of GO:0045912; is a type of regulation of galactomannan catabolic process [GO:2000991]; negatively regulates galactomannan catabolic process [GO:0051682] Definition: Any process that stops, prevents or reduces the frequency, rate or extent of galactomannan catabolic process. Sources: GOC:mengo_curators